light-activated voltage-gated calcium channel complex [GO:0008087] (cellular component) Relationships: is a type of voltage-gated calcium channel complex [GO:0005891] Also known as: light-activated voltage gated calcium channel complex, light-activated voltage-dependent calcium channel complex, light-activated voltage-sensitive calcium channel complex Definition: A protein complex that forms a transmembrane channel through which calcium ions may cross a cell membrane in response to changes in membrane potential generated in response to a light stimulus. References: PMID:9223679 Sources: GOC:mah